{
  "gene_symbol": "UBQLNL",
  "term_id": "GO:0006511",
  "term_label": "ubiquitin-dependent protein catabolic process",
  "gene_name": "Ubiquilin-like protein",
  "gene": "UniProtKB:Q8IYU4"
}